{
  "gene_symbol": "DCANP1",
  "gene": "UniProtKB:Q8TF63",
  "gene_name": "Dendritic cell nuclear protein 1",
  "term_label": "Unknown molecular function",
  "term_id": "UNKNOWN:0001"
}